{
  "gene_symbol": "SRD5A1",
  "term_label": "3-oxo-5-alpha-steroid 4-dehydrogenase activity",
  "gene_name": "3-oxo-5-alpha-steroid 4-dehydrogenase 1",
  "term_id": "GO:0003865",
  "gene": "UniProtKB:P18405"
}